{
  "gene_symbol": "PI4KA",
  "term_label": "cytoplasm",
  "term_id": "GO:0005737",
  "gene": "UniProtKB:P42356",
  "gene_name": "Phosphatidylinositol 4-kinase alpha"
}